{
  "gene": "UniProtKB:Q02790",
  "term_label": "cytosol",
  "term_id": "GO:0005829",
  "gene_symbol": "FKBP4",
  "gene_name": "Peptidyl-prolyl cis-trans isomerase FKBP4"
}